toll-like receptor 2 signaling pathway [GO:0034134] (biological process) Regulation: RO_0002211 by regulation of toll-like receptor 2 signaling pathway [GO:0034135]; negatively regulated by GO:0034136; positively regulated by GO:0034137 Subtypes: MyD88-dependent toll-like receptor 2 signaling pathway [GO:0035661] Relationships: is a type of cell surface toll-like receptor signaling pathway [GO:0140895] Definition: The series of molecular signals initiated by a ligand binding to toll-like receptor 2. Also known as: TLR2 signaling pathway, toll-like receptor 2 signalling pathway References: PMID:16551253, PMID:17328678 Sources: GOC:add